ubiquitin-like protein reader activity [GO:0140035] (molecular function) References: PMID:26060076 Relationships: is a type of GO:0030674; has part modification-dependent protein binding [GO:0140030] Note: This term should only be used when the binding is shown to require a ubiquitin-like modification in the target protein: the interaction needs to be tested with and without the PTM. The binding does not need to be at the site of ubiquitin-like modification. It may be that the modification causes a conformational change that allows binding of the protein to another region; this type of modification-dependent protein binding is valid for annotation to this term. Subtypes: GO:0140036, SUMO-modified protein reader activity [GO:0140037], GO:0141185 Definition: A molecular adaptor that recognizes and binds a target protein containing a ubiquitin-like modification and that brings the target protein into contact with another protein to allow those proteins to function in a coordinated way. Also known as: ubiquitination-like modification-dependent protein binding, ubiquitination-like protein reader activity